{
  "gene_name": "Histone H2A",
  "gene": "UniProtKB:A0A8Q3WKH5",
  "gene_symbol": "H2AL1Q",
  "term_id": "GO:0031507",
  "term_label": "heterochromatin formation"
}